{
  "term_id": "GO:0050911",
  "term_label": "detection of chemical stimulus involved in sensory perception of smell",
  "gene_symbol": "OR2B3",
  "gene_name": "Putative olfactory receptor 2B3",
  "gene": "UniProtKB:O76000"
}